{
  "gene_symbol": "NCS1",
  "term_label": "regulation of signal transduction",
  "gene_name": "Neuronal calcium sensor 1",
  "gene": "UniProtKB:P62166",
  "term_id": "GO:0009966"
}